{
  "gene": "UniProtKB:P18428",
  "term_label": "macrophage activation involved in immune response",
  "term_id": "GO:0002281",
  "gene_name": "Lipopolysaccharide-binding protein",
  "gene_symbol": "LBP"
}